mitochondrial glutamate synthase complex (NADH) [GO:0043294] (cellular component) References: PMID:7047525 Sources: GOC:jl Definition: A protein complex, found in the mitochondria, that in yeast consists of a large and a small subunit. Possesses glutamate synthase (NADH) activity. Relationships: is a type of glutamate synthase complex (NADH) [GO:0031027]; is a type of GO:0098798; BFO_0000050 GO:0005759